{
  "gene_symbol": "SPAG6",
  "term_id": "GO:0008017",
  "gene_name": "Sperm-associated antigen 6",
  "term_label": "microtubule binding",
  "gene": "UniProtKB:O75602"
}